non-canonical Wnt signaling pathway involved in heart development [GO:0061341] (biological process) Relationships: is a type of GO:0003306; is a type of GO:0035567 Definition: The series of molecular signals initiated by binding of a Wnt protein to a frizzled family receptor on the surface of the target cell, followed by propagation of the signal via effectors other than beta-catenin and contributing to the progression of the heart over time. References: PMID:16860783 Sources: GOC:dph, GOC:mtg_heart Also known as: non-canonical Wnt receptor signaling pathway involved in heart development, non-canonical Wnt receptor signalling pathway involved in heart development, non-canonical Wnt-activated signaling pathway involved in heart development Subtypes: planar cell polarity pathway involved in cardiac muscle cell fate commitment [GO:0061345]